porphyrin-containing compound biosynthetic process [GO:0006779] (biological process) Also known as: porphyrin anabolism, porphyrin biosynthesis, porphyrin biosynthetic process, porphyrin formation, porphyrin synthesis Subtypes: uroporphyrinogen III biosynthetic process [GO:0006780], succinyl-CoA pathway [GO:0006781], protoporphyrinogen IX biosynthetic process [GO:0006782], heme biosynthetic process [GO:0006783], chlorophyll biosynthetic process [GO:0015995] Relationships: is a type of porphyrin-containing compound metabolic process [GO:0006778]; is a type of GO:0033014 Definition: The chemical reactions and pathways resulting in the formation of any member of a large group of derivatives or analogs of porphyrin. Porphyrin consists of a ring of four pyrrole nuclei linked each to the next at their alpha positions through a methine group. Sources: GOC:jl, ISBN:0198506732, Wikipedia:Porphyrin#Natural_formation